positive regulation of translation in response to oxidative stress [GO:0032939] (biological process) Relationships: is a type of positive regulation of translation in response to stress [GO:0032056]; is part of cellular response to oxidative stress [GO:0034599] Sources: GOC:mah Also known as: up regulation of translation in response to oxidative stress, up-regulation of translation in response to oxidative stress, upregulation of translation in response to oxidative stress, activation of translation in response to oxidative stress, stimulation of translation in response to oxidative stress Definition: Any process that activates or increases the frequency, rate or extent of translation as a result of oxidative stress, a state often resulting from exposure to high levels of reactive oxygen species, e.g. superoxide anions, hydrogen peroxide (H2O2), and hydroxyl radicals.